cell proliferation involved in kidney development [GO:0072111] (biological process) Sources: GOC:mtg_kidney_jan10 Regulation: regulated by GO:1901722; negatively regulated by negative regulation of cell proliferation involved in kidney development [GO:1901723]; positively regulated by positive regulation of cell proliferation involved in kidney development [GO:1901724] Definition: The multiplication or reproduction of cells, resulting in the expansion of the population in the kidney. Relationships: is a type of cell population proliferation [GO:0008283]; is part of kidney development [GO:0001822] Subtypes: GO:0039015, cell proliferation involved in mesonephros development [GO:0061209], glomerular mesangial cell proliferation [GO:0072110], GO:0072122, GO:0072135, cell proliferation involved in metanephros development [GO:0072203]